{
  "term_id": "GO:0005929",
  "gene_name": "Intraflagellar transport protein 27 homolog",
  "gene": "UniProtKB:Q9BW83",
  "term_label": "cilium",
  "gene_symbol": "IFT27"
}